regulation of positive thymic T cell selection [GO:1902232] (biological process) References: PMID:22080863 Sources: GOC:TermGenie Relationships: is_a regulation of T cell differentiation in thymus [GO:0033081]; RO_0002211 positive thymic T cell selection [GO:0045059] Definition: Any process that modulates the frequency, rate or extent of positive thymic T cell selection. Subtypes: negative regulation of positive thymic T cell selection [GO:1902233], positive regulation of positive thymic T cell selection [GO:1902234] Also known as: regulation of positive thymic T lymphocyte selection, regulation of positive thymic T-cell selection, regulation of positive thymic T-lymphocyte selection